L-cysteine catabolic process to pyruvate, using cysteine dioxygenase [GO:0019451] (biological process) Sources: GOC:jl Also known as: L-cysteine breakdown to pyruvate, using cysteine dioxygenase, L-cysteine degradation to pyruvate, using cysteine dioxygenase Definition: The chemical reactions and pathways resulting in the breakdown into pyruvate of L-cystine, catalyzed by the enzyme cysteine dioxygenase (EC:1.13.11.20). Relationships: is a type of GO:0019450; has part cysteine dioxygenase activity [GO:0017172]